{
  "gene_name": "Cilia- and flagella-associated protein 47",
  "term_label": "cilium assembly",
  "gene_symbol": "CFAP47",
  "term_id": "GO:0060271",
  "gene": "UniProtKB:Q6ZTR5"
}